rhoptry lumen [GO:0034591] (cellular component) References: PMID:17997128 Sources: GOC:rph Definition: The volume enclosed by the rhoptry membrane. Relationships: is a type of GO:0043233; is part of rhoptry [GO:0020008]